{
  "term_label": "GTP binding",
  "gene_symbol": "RAB2B",
  "term_id": "GO:0005525",
  "gene": "UniProtKB:Q8WUD1",
  "gene_name": "Ras-related protein Rab-2B"
}